{
  "gene": "UniProtKB:O15155",
  "term_label": "SNARE complex",
  "gene_name": "BET1 homolog",
  "gene_symbol": "BET1",
  "term_id": "GO:0031201"
}